{
  "term_label": "calcium-dependent cell-cell adhesion",
  "gene": "UniProtKB:Q9H159",
  "gene_name": "Cadherin-19",
  "gene_symbol": "CDH19",
  "term_id": "GO:0016339"
}